{
  "term_label": "activation of innate immune response",
  "gene_name": "NACHT, LRR and PYD domains-containing protein 1",
  "term_id": "GO:0002218",
  "gene": "UniProtKB:Q9C000",
  "gene_symbol": "NLRP1"
}